L-arabinitol 4-dehydrogenase activity [GO:0050019] (molecular function) Relationships: is a type of GO:0016616 Definition: Catalysis of the reaction: L-arabinitol + NAD+ = L-xylulose + H+ + NADH. Sources: EC:1.1.1.12, RHEA:16381